{
  "gene": "UniProtKB:Q9BZG2",
  "term_label": "receptor tyrosine kinase binding",
  "gene_name": "Testicular acid phosphatase",
  "gene_symbol": "ACP4",
  "term_id": "GO:0030971"
}